{
  "term_label": "positive regulation of MAPK cascade",
  "term_id": "GO:0043410",
  "gene_name": "Alpha-1B adrenergic receptor",
  "gene": "UniProtKB:P35368",
  "gene_symbol": "ADRA1B"
}